{
  "gene": "UniProtKB:Q9HC35",
  "gene_name": "Echinoderm microtubule-associated protein-like 4",
  "gene_symbol": "EML4",
  "term_label": "microtubule binding",
  "term_id": "GO:0008017"
}